{
  "gene_symbol": "UFD1",
  "gene_name": "Ubiquitin recognition factor in ER-associated degradation protein 1",
  "term_id": "GO:0031593",
  "gene": "UniProtKB:Q92890",
  "term_label": "polyubiquitin modification-dependent protein binding"
}